{
  "gene_symbol": "PMFBP1",
  "gene_name": "Polyamine-modulated factor 1-binding protein 1",
  "term_label": "Unknown molecular function",
  "term_id": "UNKNOWN:0001",
  "gene": "UniProtKB:Q8TBY8"
}